RNA helicase inhibitor activity [GO:1990119] (molecular function) References: PMID:23721653 Sources: GOC:rb Definition: Binds to and stops, prevents or reduces the activity of an RNA helicase. Relationships: is a type of GO:0004857; is a type of ATPase inhibitor activity [GO:0042030]; negatively regulates RNA helicase activity [GO:0003724] Also known as: ATP-dependent RNA helicase inhibitor activity